{
  "term_label": "Unknown molecular function",
  "gene_name": "Serine_threonine-protein phosphatase CPPED1",
  "gene_symbol": "CPPED1",
  "gene": "UniProtKB:Q9BRF8",
  "term_id": "UNKNOWN:0001"
}